response to water [GO:0009415] (biological process) Also known as: response to water stimulus Sources: GOC:jl Definition: Any process that results in a change in state or activity of a cell or an organism (in terms of movement, secretion, enzyme production, gene expression, etc.) as a result of a stimulus reflecting the presence, absence, or concentration of water. Subtypes: response to humidity [GO:0009270], response to flooding [GO:0009413], response to water deprivation [GO:0009414], response to deep water [GO:0030912], response to hydrostatic pressure [GO:0051599], cellular response to water stimulus [GO:0071462] Relationships: is a type of response to acid chemical [GO:0001101]; is a type of GO:0009628; is_a response to oxygen-containing compound [GO:1901700]